{
  "gene": "UniProtKB:P61254",
  "gene_name": "Large ribosomal subunit protein uL24",
  "term_id": "GO:0002181",
  "term_label": "cytoplasmic translation",
  "gene_symbol": "RPL26"
}